{
  "term_id": "UNKNOWN:0003",
  "gene_symbol": "MMP1",
  "gene": "UniProtKB:P03956",
  "gene_name": "Interstitial collagenase",
  "term_label": "Unknown cellular component"
}